{
  "gene": "UniProtKB:Q6ZS62",
  "term_id": "UNKNOWN:0003",
  "gene_name": "Colorectal cancer-associated protein 1",
  "gene_symbol": "COLCA1",
  "term_label": "Unknown cellular component"
}